{
  "term_id": "GO:0001540",
  "gene_symbol": "APBA1",
  "gene_name": "Amyloid-beta A4 precursor protein-binding family A member 1",
  "gene": "UniProtKB:Q02410",
  "term_label": "amyloid-beta binding"
}